{
  "term_id": "GO:0006366",
  "gene_name": "TFIIA-alpha and beta-like factor",
  "term_label": "transcription by RNA polymerase II",
  "gene": "UniProtKB:Q9UNN4",
  "gene_symbol": "GTF2A1L"
}